{
  "gene_symbol": "ABCA6",
  "term_label": "lipid transporter activity",
  "gene_name": "ATP-binding cassette sub-family A member 6",
  "gene": "UniProtKB:Q8N139",
  "term_id": "GO:0005319"
}